cardiac muscle progenitor cell migration to the midline involved in heart field formation [GO:0003261] (biological process) Definition: The orderly movement of a myocardial progenitor cell toward the midline to form the heart field. Cardiac muscle progenitor cells are non-terminally differentiated, mesoderm-derived cells that are committed to differentiate into myocardial cells of the heart. Also known as: myocardial progenitor cell midline convergence Sources: GOC:mtg_heart Relationships: is_a cardioblast migration to the midline involved in heart field formation [GO:0060975]